positive regulation of small molecule metabolic process [GO:0062013] (biological process) Also known as: positive regulation of small molecule metabolism Subtypes: GO:0010372, GO:0010907, positive regulation of penicillin metabolic process [GO:0033246], positive regulation of acetate catabolic process [GO:0045754], positive regulation of fatty acid metabolic process [GO:0045923], GO:0045979, GO:0045981, GO:0045983, GO:0045985, positive regulation of ecdysteroid biosynthetic process [GO:0045998], positive regulation of vitamin metabolic process [GO:0046136], positive regulation of taurine biosynthetic process [GO:0062090], positive regulation of L-glutamine biosynthetic process [GO:0062134], positive regulation of bile acid biosynthetic process [GO:0070859], GO:0090205, positive regulation of L-tryptophan metabolic process [GO:0090358], positive regulation of (R)-mevalonic acid biosynthetic process [GO:0106109], GO:0106280, positive regulation of histidine biosynthetic process [GO:0120215], positive regulation of pyruvate decarboxylation to acetyl-CoA [GO:0140176], positive regulation of N-acetylmuramic acid catabolic process [GO:0160159], positive regulation of arginine biosynthetic process [GO:1900080], GO:1900179, positive regulation of xanthone-containing compound biosynthetic process [GO:1900185], positive regulation of methane biosynthetic process from formic acid [GO:1900341], positive regulation of asperthecin biosynthetic process [GO:1900381], positive regulation of alcohol catabolic process [GO:1900421], GO:1900486, positive regulation of xylose catabolic process to ethanol [GO:1900517], positive regulation of emericellamide biosynthetic process [GO:1900660], positive regulation of emodin biosynthetic process [GO:1900666], positive regulation of endocrocin biosynthetic process [GO:1900669], positive regulation of fumonisin biosynthetic process [GO:1900685], positive regulation of gerfelin biosynthetic process [GO:1900688], GO:1900700, positive regulation of tensidol A biosynthetic process [GO:1900709], positive regulation of tensidol B biosynthetic process [GO:1900712], positive regulation of helvolic acid biosynthetic process [GO:1900842], positive regulation of monodictyphenone biosynthetic process [GO:1900845], positive regulation of naphtho-gamma-pyrone biosynthetic process [GO:1900848], positive regulation of pseurotin A biosynthetic process [GO:1900851], positive regulation of terrequinone A biosynthetic process [GO:1900854], positive regulation of sarcinapterin biosynthetic process [GO:1900973], positive regulation of tatiopterin biosynthetic process [GO:1900976], positive regulation of tetrapyrrole biosynthetic process from glutamate [GO:1901412], positive regulation of tetrapyrrole biosynthetic process from glycine and succinyl-CoA [GO:1901415], positive regulation of ferulate catabolic process [GO:1901468], positive regulation of homoserine biosynthetic process [GO:1901712], positive regulation of urea catabolic process [GO:1901714], positive regulation of gamma-aminobutyric acid catabolic process [GO:1901717], positive regulation of fumagillin biosynthetic process [GO:1902092], GO:1902932, positive regulation of L-dopa biosynthetic process [GO:1903197], positive regulation of citrulline biosynthetic process [GO:1903250], positive regulation of ornithine catabolic process [GO:1903268], positive regulation of androst-4-ene-3,17-dione biosynthetic process [GO:1903456], positive regulation of ubiquinone biosynthetic process [GO:1904775], positive regulation of quinolinate biosynthetic process [GO:1904986], GO:2000184, GO:2000876, positive regulation of L-proline catabolic process to L-glutamate [GO:2001158], positive regulation of glycolytic fermentation to ethanol [GO:2001172], positive regulation of lysine biosynthetic process via alpha-aminoadipate and saccharopine [GO:2001196], positive regulation of ammonia assimilation cycle [GO:2001250], positive regulation of L-leucine biosynthetic process [GO:2001278] Definition: Any process that activates or increases the frequency, rate or extent of a small molecule metabolic process. Relationships: is a type of GO:0009893; is a type of regulation of small molecule metabolic process [GO:0062012]; positively regulates GO:0044281 Sources: GOC:vw